{
  "term_label": "Unknown biological process",
  "gene": "UniProtKB:Q8WVE0",
  "gene_symbol": "EEF1AKMT1",
  "gene_name": "EEF1A lysine methyltransferase 1",
  "term_id": "UNKNOWN:0002"
}